{
  "gene": "UniProtKB:P56730",
  "gene_name": "Neurotrypsin",
  "gene_symbol": "PRSS12",
  "term_id": "GO:0043195",
  "term_label": "terminal bouton"
}